{
  "gene": "UniProtKB:Q9Y334",
  "term_id": "UNKNOWN:0003",
  "gene_symbol": "VWA7",
  "gene_name": "von Willebrand factor A domain-containing protein 7",
  "term_label": "Unknown cellular component"
}